{
  "term_label": "positive regulation of canonical NF-kappaB signal transduction",
  "gene": "UniProtKB:O15205",
  "term_id": "GO:0043123",
  "gene_name": "Ubiquitin D",
  "gene_symbol": "UBD"
}